interleukin-15 production [GO:0032618] (biological process) Relationships: is a type of GO:0001816 Sources: GOC:mah Definition: The appearance of interleukin-15 due to biosynthesis or secretion following a cellular stimulus, resulting in an increase in its intracellular or extracellular levels. Also known as: IL-15 production, interleukin-15 biosynthetic process, interleukin-15 secretion Regulation: RO_0002211 by regulation of interleukin-15 production [GO:0032658]; negatively regulated by negative regulation of interleukin-15 production [GO:0032698]; positively regulated by positive regulation of interleukin-15 production [GO:0032738]